acropetal auxin transport [GO:0010541] (biological process) Definition: The unidirectional movement of auxin from the base towards the apex of an organ, including the shoot, leaf, primary root, or lateral root. Relationships: is a type of auxin polar transport [GO:0009926] References: PMID:10677441